laminin-7 complex [GO:0005612] (cellular component) Definition: A laminin complex composed of alpha3, beta2 and gamma1 polypeptide chains. References: PMID:10842354 Sources: GOC:jl Also known as: laminin-7A, laminin-321 complex Relationships: is a type of laminin complex [GO:0043256]